{
  "term_label": "chromatin",
  "gene_symbol": "TCF7",
  "term_id": "GO:0000785",
  "gene": "UniProtKB:P36402",
  "gene_name": "Transcription factor 7"
}